negative regulation of xanthone-containing compound biosynthetic process [GO:1900184] (biological process) Sources: GOC:TermGenie, GOC:di Definition: Any process that stops, prevents or reduces the frequency, rate or extent of xanthone-containing compound biosynthetic process. Relationships: is a type of negative regulation of biosynthetic process [GO:0009890]; is a type of negative regulation of small molecule metabolic process [GO:0062014]; is a type of regulation of xanthone-containing compound biosynthetic process [GO:1900183]; negatively regulates GO:2001307 Also known as: down regulation of xanthone-containing compound anabolism, down regulation of xanthone-containing compound biosynthesis, down regulation of xanthone-containing compound biosynthetic process, down regulation of xanthone-containing compound formation, down regulation of xanthone-containing compound synthesis, down-regulation of xanthone-containing compound anabolism, down-regulation of xanthone-containing compound biosynthesis, down-regulation of xanthone-containing compound biosynthetic process, down-regulation of xanthone-containing compound formation, down-regulation of xanthone-containing compound synthesis, downregulation of xanthone-containing compound anabolism, downregulation of xanthone-containing compound biosynthesis, downregulation of xanthone-containing compound biosynthetic process, downregulation of xanthone-containing compound formation, downregulation of xanthone-containing compound synthesis, inhibition of xanthone-containing compound anabolism, inhibition of xanthone-containing compound biosynthesis, inhibition of xanthone-containing compound formation, inhibition of xanthone-containing compound synthesis, negative regulation of xanthone-containing compound anabolism, negative regulation of xanthone-containing compound biosynthesis, negative regulation of xanthone-containing compound formation, negative regulation of xanthone-containing compound synthesis, negative regulation of xanthones anabolism, down regulation of xanthone biosynthesis, down regulation of xanthone biosynthetic process, down-regulation of xanthone biosynthesis, down-regulation of xanthone biosynthetic process, downregulation of xanthone biosynthesis, downregulation of xanthone biosynthetic process, inhibition of xanthone biosynthesis, inhibition of xanthone biosynthetic process, inhibition of xanthone-containing compound biosynthetic process, negative regulation of xanthone biosynthesis, negative regulation of xanthone biosynthetic process Subtypes: negative regulation of emericellin biosynthetic process [GO:1900835]